{
  "gene_name": "Protein BEAN1",
  "gene": "UniProtKB:Q3B7T3",
  "term_id": "UNKNOWN:0002",
  "term_label": "Unknown biological process",
  "gene_symbol": "BEAN1"
}